cell proliferation involved in heart valve morphogenesis [GO:0003249] (biological process) Relationships: is a type of GO:0061323; is a type of cell proliferation involved in heart valve development [GO:2000793]; is part of heart valve morphogenesis [GO:0003179] Definition: The multiplication or reproduction of cells that contributes to the shaping of a heart valve. Sources: GOC:mtg_heart Regulation: regulated by regulation of cell proliferation involved in heart valve morphogenesis [GO:0003250]; positively regulated by positive regulation of cell proliferation involved in heart valve morphogenesis [GO:0003251]; negatively regulated by negative regulation of cell proliferation involved in heart valve morphogenesis [GO:0003252]